glucose-6-phosphate dehydrogenase activity [GO:0004345] (molecular function) Also known as: 6-phosphoglucose dehydrogenase activity, D-glucose 6-phosphate dehydrogenase activity, G6PDH, NADP-dependent glucose 6-phosphate dehydrogenase activity, NADP-glucose-6-phosphate dehydrogenase activity, glucose 6-phosphate dehydrogenase (NADP) activity, glucose-6-phosphate 1-dehydrogenase activity, 6-phosphoglucose dehydrogenas, D-glucose-6-phosphate:NADP+ 1-oxidoreductase activity, Entner-doudoroff enzyme, G6PD activity, GDH, Zwischenferment Relationships: is_a oxidoreductase activity, acting on the CH-OH group of donors, NAD or NADP as acceptor [GO:0016616] Sources: EC:1.1.1.49 Definition: Catalysis of the reaction: D-glucose 6-phosphate + NADP+ = D-glucono-1,5-lactone 6-phosphate + NADPH + H+.